{
  "term_label": "1-phosphatidylinositol-4-phosphate 3-kinase activity",
  "gene": "UniProtKB:P42338",
  "gene_symbol": "PIK3CB",
  "term_id": "GO:0035005",
  "gene_name": "Phosphatidylinositol 4,5-bisphosphate 3-kinase catalytic subunit beta isoform"
}